{
  "term_id": "GO:2000641",
  "gene_symbol": "DENND10",
  "gene_name": "DENN domain-containing protein 10",
  "gene": "UniProtKB:Q8TCE6",
  "term_label": "regulation of early endosome to late endosome transport"
}